{
  "gene": "UniProtKB:Q86VS8",
  "term_label": "centrosome",
  "term_id": "GO:0005813",
  "gene_name": "Protein Hook homolog 3",
  "gene_symbol": "HOOK3"
}